{
  "term_label": "regulation of calcium ion-dependent exocytosis",
  "term_id": "GO:0017158",
  "gene": "UniProtKB:Q9BQG1",
  "gene_symbol": "SYT3",
  "gene_name": "Synaptotagmin-3"
}